glycolate biosynthetic process [GO:0046295] (biological process) Subtypes: GO:0036529 Definition: The chemical reactions and pathways resulting in the formation of glycolate, the anion of hydroxyethanoic acid (glycolic acid). Relationships: is a type of glycolate metabolic process [GO:0009441]; is a type of primary alcohol biosynthetic process [GO:0034309]; is a type of monocarboxylic acid biosynthetic process [GO:0072330] Sources: GOC:ai Also known as: glycolate anabolism, glycolate biosynthesis, glycolate formation, glycolate synthesis